{
  "gene_symbol": "JAK3",
  "term_id": "GO:0005829",
  "term_label": "cytosol",
  "gene_name": "Tyrosine-protein kinase JAK3",
  "gene": "UniProtKB:P52333"
}